{
  "term_id": "UNKNOWN:0003",
  "term_label": "Unknown cellular component",
  "gene_name": "Putative uncharacterized protein encoded by MIR1915-HG",
  "gene_symbol": "MIR1915HG",
  "gene": "UniProtKB:Q5T4H9"
}